{
  "term_label": "cell migration",
  "gene_name": "Cadherin-1",
  "term_id": "GO:0016477",
  "gene_symbol": "CDH1",
  "gene": "UniProtKB:P12830"
}